{
  "gene_name": "Keratin, type I cytoskeletal 25",
  "gene_symbol": "KRT25",
  "term_label": "keratin filament",
  "term_id": "GO:0045095",
  "gene": "UniProtKB:Q7Z3Z0"
}